{
  "term_label": "P-body",
  "gene_symbol": "PAN2",
  "gene_name": "PAN2-PAN3 deadenylation complex catalytic subunit PAN2",
  "term_id": "GO:0000932",
  "gene": "UniProtKB:Q504Q3"
}